{
  "gene": "UniProtKB:Q15390",
  "gene_symbol": "MTFR1",
  "term_label": "mitochondrial fission",
  "gene_name": "Mitochondrial fission regulator 1",
  "term_id": "GO:0000266"
}